neuromedin U receptor binding [GO:0042922] (molecular function) Relationships: is a type of GO:0071855 Definition: Binding to one or more specific sites on a neuromedin U receptor. Subtypes: type 1 neuromedin U receptor binding [GO:0031839], type 2 neuromedin U receptor binding [GO:0031840] References: PMID:10899166 Sources: GOC:jl